{
  "gene_name": "Cation channel sperm-associated targeting subunit tau",
  "gene": "UniProtKB:Q53TS8",
  "term_id": "UNKNOWN:0002",
  "gene_symbol": "C2CD6",
  "term_label": "Unknown biological process"
}